{
  "gene": "UniProtKB:Q8TEJ3",
  "term_label": "positive regulation of JNK cascade",
  "gene_symbol": "SH3RF3",
  "gene_name": "E3 ubiquitin-protein ligase SH3RF3",
  "term_id": "GO:0046330"
}